precorrin-2 C20-methyltransferase activity [GO:0030788] (molecular function) Also known as: S-adenosyl-L-methionine--precorrin-2 methyltransferase activity, S-adenosyl-L-methionine:precorrin-4 C20-methyltransferase activity Relationships: is a type of S-adenosylmethionine-dependent methyltransferase activity [GO:0008757] Definition: Catalysis of the reaction: S-adenosyl-L-methionine + precorrin-2 = S-adenosyl-L-homocysteine + H+ + precorrin-3A. Sources: EC:2.1.1.130, RHEA:16841